mucosal tolerance induction [GO:0002427] (biological process) Definition: Tolerance induction taking place in the mucosal tissues. Relationships: is_a GO:0002385; is a type of GO:0002462 Sources: GOC:jal Subtypes: GO:0002401, tolerance induction in urogenital tract [GO:0002425]